{
  "gene_symbol": "CDNF",
  "gene": "UniProtKB:Q49AH0",
  "term_id": "UNKNOWN:0001",
  "gene_name": "Cerebral dopamine neurotrophic factor",
  "term_label": "Unknown molecular function"
}